negative regulation of translation [GO:0017148] (biological process) Relationships: is a type of regulation of translation [GO:0006417]; is_a negative regulation of gene expression [GO:0010629]; is a type of GO:0051248; negatively regulates translation [GO:0006412] Subtypes: GO:0007319, negative regulation of translation in response to stress [GO:0032055], miRNA-mediated gene silencing by inhibition of translation [GO:0035278], negative regulation of translational elongation [GO:0045900], negative regulation of translational fidelity [GO:0045902], negative regulation of translational termination [GO:0045904], negative regulation of translational initiation [GO:0045947], negative regulation of mitochondrial translation [GO:0070130], GO:0070549, ribosome hibernation [GO:0141014], negative regulation of cytoplasmic translation [GO:2000766] Definition: Any process that stops, prevents, or reduces the frequency, rate or extent of the chemical reactions and pathways resulting in the formation of proteins by the translation of mRNA or circRNA. Also known as: down regulation of protein biosynthetic process, down-regulation of protein biosynthetic process, downregulation of protein biosynthetic process, negative regulation of protein anabolism, negative regulation of protein biosynthesis, negative regulation of protein biosynthetic process, negative regulation of protein formation, negative regulation of protein synthesis, inhibition of protein biosynthetic process, protein biosynthesis inhibitor activity, protein biosynthetic process inhibitor activity Sources: GOC:isa_complete